positive regulation of skeletal muscle tissue growth [GO:0048633] (biological process) Definition: Any process that activates, maintains or increases the rate of skeletal muscle growth. References: PMID:15726494, PMID:15907921 Sources: GOC:lm Also known as: up regulation of skeletal muscle growth, up-regulation of skeletal muscle growth, upregulation of skeletal muscle growth, activation of skeletal muscle growth, stimulation of skeletal muscle growth Relationships: is a type of regulation of skeletal muscle tissue growth [GO:0048631]; is a type of positive regulation of developmental growth [GO:0048639]; is a type of positive regulation of skeletal muscle tissue development [GO:0048643]; positively regulates skeletal muscle tissue growth [GO:0048630]